{
  "gene_symbol": "SLC26A4",
  "term_label": "chloride:bicarbonate antiporter activity",
  "gene": "UniProtKB:O43511",
  "gene_name": "Pendrin",
  "term_id": "GO:0140900"
}